peptidyl-thiazoline dehydrogenase activity [GO:0018136] (molecular function) Definition: Catalysis of the reduction of a peptide-linked thiazoline to thiazole. References: PMID:19058272 Sources: GOC:mah Relationships: is a type of oxidoreductase activity, acting on the CH-CH group of donors [GO:0016627]